positive regulation of release of cytochrome c from mitochondria [GO:0090200] (biological process) Note: The release of cytochrome c from mitochondria is a central event in the signaling phase of the apoptotic process, and it is often used by researchers to monitor this type of cell death. Any event that induces apoptosis will at some point induce the release of cytochrome c from mitochondria. Therefore, this term should only be used to annotate gene products that directly and positively regulate this process. Definition: Any process that increases the rate, frequency or extent of release of cytochrome c from mitochondria, the process in which cytochrome c is enabled to move from the mitochondrial intermembrane space into the cytosol, which is an early step in apoptosis and leads to caspase activation. Relationships: is a type of positive regulation of organelle organization [GO:0010638]; is a type of GO:0090199; positively regulates release of cytochrome c from mitochondria [GO:0001836] Sources: GOC:BHF, GOC:dph, GOC:mtg_apoptosis, GOC:tb